{
  "term_label": "acetylesterase activity",
  "gene": "UniProtKB:P08910",
  "gene_name": "Monoacylglycerol lipase ABHD2",
  "term_id": "GO:0008126",
  "gene_symbol": "ABHD2"
}